{
  "gene_name": "Lactadherin",
  "gene_symbol": "MFGE8",
  "term_label": "Unknown biological process",
  "gene": "UniProtKB:Q08431",
  "term_id": "UNKNOWN:0002"
}